{
  "gene": "UniProtKB:Q96LI9",
  "gene_symbol": "CXorf58",
  "term_label": "Unknown molecular function",
  "term_id": "UNKNOWN:0001",
  "gene_name": "Uncharacterized protein CXorf58"
}